{
  "term_label": "regulation of transcription by RNA polymerase II",
  "gene": "UniProtKB:P18850",
  "term_id": "GO:0006357",
  "gene_name": "Cyclic AMP-dependent transcription factor ATF-6 alpha",
  "gene_symbol": "ATF6"
}